delphinidin 3-O-glucoside biosynthetic process [GO:0033486] (biological process) Definition: The chemical reactions and pathways resulting in the formation of delphinidin 3-O-glucoside, a basic, water-soluble anthocyanin responsible for blue coloration of flowers and fruits. Relationships: is a type of GO:0009813; is a type of beta-glucoside biosynthetic process [GO:1901806] Sources: GOC:mah, MetaCyc:PWY-5153 Also known as: delphinidin 3-O-glucoside anabolism, delphinidin 3-O-glucoside biosynthesis, delphinidin 3-O-glucoside formation, delphinidin 3-O-glucoside synthesis